{
  "gene_name": "C-X-C motif chemokine 2",
  "term_label": "Unknown molecular function",
  "term_id": "UNKNOWN:0001",
  "gene": "UniProtKB:P19875",
  "gene_symbol": "CXCL2"
}